positive regulation of sensory perception of bitter taste [GO:1904662] (biological process) Also known as: positive regulation of bitter taste perception, up regulation of bitter taste perception, up regulation of sensory perception of bitter taste, up-regulation of bitter taste perception, up-regulation of sensory perception of bitter taste, upregulation of bitter taste perception, upregulation of sensory perception of bitter taste, activation of bitter taste perception, activation of sensory perception of bitter taste Definition: Any process that activates or increases the frequency, rate or extent of sensory perception of bitter taste. References: PMID:1716172 Sources: GOC:TermGenie, GOC:mr, GO_REF:0000058 Relationships: is a type of positive regulation of nervous system process [GO:0031646]; is a type of GO:1904660; RO_0002213 sensory perception of bitter taste [GO:0050913]